neurotransmitter receptor complex [GO:0098878] (CC) Relationships: is a type of plasma membrane signaling receptor complex [GO:0098802] Definition: Any protein complex that is capable of functioning as a neurotransmitter receptor. Sources: GOC:dos Subtypes: ionotropic glutamate receptor complex [GO:0008328], serotonin-activated cation-selective channel complex [GO:1904602]